{
  "gene_name": "Ryanodine receptor 3",
  "term_id": "GO:0033017",
  "gene": "UniProtKB:Q15413",
  "gene_symbol": "RYR3",
  "term_label": "sarcoplasmic reticulum membrane"
}